{
  "term_label": "mitochondrion",
  "gene_symbol": "MCCC2",
  "gene_name": "Methylcrotonoyl-CoA carboxylase beta chain, mitochondrial",
  "gene": "UniProtKB:Q9HCC0",
  "term_id": "GO:0005739"
}